{
  "gene": "UniProtKB:Q8TAA5",
  "term_id": "GO:0000774",
  "term_label": "adenyl-nucleotide exchange factor activity",
  "gene_name": "GrpE protein homolog 2, mitochondrial",
  "gene_symbol": "GRPEL2"
}